{
  "term_id": "GO:0000070",
  "term_label": "mitotic sister chromatid segregation",
  "gene_symbol": "ZWINT",
  "gene": "UniProtKB:O95229",
  "gene_name": "ZW10 interactor"
}